glycosphingolipid biosynthetic process [GO:0006688] (biological process) Relationships: is a type of GO:0006687; is a type of glycolipid biosynthetic process [GO:0009247]; is a type of sphingolipid biosynthetic process [GO:0030148] Subtypes: lactosylceramide biosynthetic process [GO:0001572], GO:0001574, globoside biosynthetic process [GO:0001576], glucosylceramide biosynthetic process [GO:0006679], galactosylceramide biosynthetic process [GO:0006682], mannosyl-inositol phosphorylceramide biosynthetic process [GO:0051999], arthro-series glucosylceramide biosynthetic process [GO:0140269], isogloboside biosynthetic process [GO:1990387] Also known as: glycosphingolipid anabolism, glycosphingolipid biosynthesis, glycosphingolipid formation, glycosphingolipid synthesis, glycosylceramide biosynthetic process References: PMID:35536927 Definition: The chemical reactions and pathways resulting in the formation of a glycosphingolipid, a compound composed of a ceramide backbone covalently linked to at least one carbohydrate moiety.